hydrocarbon catabolic process [GO:0120253] (biological process) Sources: GOC:krc, Wikipedia:Hydrocarbon Subtypes: GO:0018915, fluorene catabolic process [GO:0019429], GO:0042184, toluene catabolic process [GO:0042203], styrene catabolic process [GO:0042207], phenanthrene catabolic process [GO:0042216], alkane catabolic process [GO:0043448], GO:0043451, alkyne catabolic process [GO:0043454], terpene catabolic process [GO:0046247], benzene catabolic process [GO:1900996], naphthalene catabolic process [GO:1901170] Also known as: hydrocarbon breakdown, hydrocarbon catabolism, hydrocarbon degradation Definition: The chemical reactions and pathways resulting in the breakdown of a hydrocarbon, a compound consisting of carbon and hydrogen only. Relationships: is_a catabolic process [GO:0009056]; is a type of hydrocarbon metabolic process [GO:0120252]